{
  "term_id": "GO:0001508",
  "term_label": "action potential",
  "gene_symbol": "KCNA5",
  "gene_name": "Potassium voltage-gated channel subfamily A member 5",
  "gene": "UniProtKB:P22460"
}